{
  "term_label": "Unknown molecular function",
  "term_id": "UNKNOWN:0001",
  "gene_symbol": "KLHDC7A",
  "gene": "UniProtKB:Q5VTJ3",
  "gene_name": "Kelch domain-containing protein 7A"
}